{
  "gene_symbol": "IL23R",
  "term_id": "GO:0072536",
  "gene": "UniProtKB:Q5VWK5",
  "gene_name": "Interleukin-23 receptor",
  "term_label": "interleukin-23 receptor complex"
}